{
  "gene": "UniProtKB:A6NCE7",
  "gene_name": "Microtubule-associated proteins 1A_1B light chain 3 beta 2",
  "term_label": "autophagosome membrane",
  "term_id": "GO:0000421",
  "gene_symbol": "MAP1LC3B2"
}